{
  "term_id": "GO:0004879",
  "gene_name": "Bile acid receptor",
  "gene_symbol": "NR1H4",
  "gene": "UniProtKB:Q96RI1",
  "term_label": "nuclear receptor activity"
}